{
  "term_label": "Unknown biological process",
  "gene": "UniProtKB:Q6AI12",
  "gene_name": "Ankyrin repeat domain-containing protein 40",
  "term_id": "UNKNOWN:0002",
  "gene_symbol": "ANKRD40"
}